ABC-type ferric hydroxamate transporter activity [GO:0015625] (molecular function) Definition: Enables the transfer of a solute or solutes from one side of a membrane to the other according to the reaction: ATP + H2O + ferric-hydroxamate(out) = ADP + phosphate + ferric-hydroxamate(in). References: PMID:1551849 Also known as: ATP-dependent iron-chelate transporter activity, ATPase-coupled iron-chelate transporter activity, ferric-hydroxamate porter activity, ferric-hydroxamate transmembrane transporter activity, iron-chelate-transporting ATPase activity, ATP-dependent ferric-hydroxamate transmembrane transporter activity, ferric-hydroxamate-transporting ATPase activity, ferric-hydroxamate ABC transporter, ATPase-coupled ferric-hydroxamate transmembrane transporter activity Relationships: is a type of GO:0015603; is a type of GO:0140359